{
  "gene_name": "Induced myeloid leukemia cell differentiation protein Mcl-1",
  "gene": "UniProtKB:Q07820",
  "term_id": "GO:0005741",
  "gene_symbol": "MCL1",
  "term_label": "mitochondrial outer membrane"
}